{
  "gene_name": "Probable cation-transporting ATPase 13A5",
  "term_id": "GO:0006874",
  "gene_symbol": "ATP13A5",
  "gene": "UniProtKB:Q4VNC0",
  "term_label": "intracellular calcium ion homeostasis"
}